{
  "term_label": "inhibitory synapse assembly",
  "term_id": "GO:1904862",
  "gene_name": "Gamma-aminobutyric acid receptor subunit alpha-6",
  "gene_symbol": "GABRA6",
  "gene": "UniProtKB:Q16445"
}